aryl-aldehyde oxidase activity [GO:0018488] (molecular function) Subtypes: abscisic aldehyde oxidase activity [GO:0010293], GO:0050302 Definition: Catalysis of the reaction: an aromatic aldehyde + O2 + H2O = an aromatic acid + hydrogen peroxide. Sources: EC:1.2.3.9 Relationships: is_a aldehyde oxidase activity [GO:0004031] Also known as: aryl-aldehyde:oxygen oxidoreductase activity